{
  "gene": "UniProtKB:O95267",
  "term_label": "B cell activation",
  "gene_symbol": "RASGRP1",
  "gene_name": "RAS guanyl-releasing protein 1",
  "term_id": "GO:0042113"
}